{
  "gene_symbol": "VILL",
  "gene_name": "Villin-like protein",
  "gene": "UniProtKB:O15195",
  "term_id": "GO:0051016",
  "term_label": "barbed-end actin filament capping"
}